{
  "term_id": "GO:0140861",
  "gene_symbol": "A8MVJ9",
  "term_label": "DNA repair-dependent chromatin remodeling",
  "gene_name": "Putative histone PARylation factor 1-like",
  "gene": "UniProtKB:A8MVJ9"
}